{
  "gene_name": "Heat shock 70 kDa protein 13",
  "term_label": "nucleus",
  "gene_symbol": "HSPA13",
  "term_id": "GO:0005634",
  "gene": "UniProtKB:P48723"
}